{
  "term_label": "respiratory chain complex III",
  "gene": "UniProtKB:P14927",
  "term_id": "GO:0045275",
  "gene_symbol": "UQCRB",
  "gene_name": "Cytochrome b-c1 complex subunit 7"
}